{
  "gene_symbol": "LINC01555",
  "gene_name": "Putative uncharacterized protein encoded by LINC01555",
  "gene": "UniProtKB:Q8NAE3",
  "term_label": "Unknown cellular component",
  "term_id": "UNKNOWN:0003"
}